{
  "term_id": "GO:0003924",
  "gene_symbol": "RAB36",
  "term_label": "GTPase activity",
  "gene_name": "Ras-related protein Rab-36",
  "gene": "UniProtKB:O95755"
}